{
  "gene_symbol": "TRIM31",
  "gene": "UniProtKB:Q9BZY9",
  "term_id": "GO:0061630",
  "gene_name": "E3 ubiquitin-protein ligase TRIM31",
  "term_label": "ubiquitin protein ligase activity"
}